{
  "term_label": "structural constituent of ribosome",
  "gene_symbol": "RPLP0P6",
  "term_id": "GO:0003735",
  "gene": "UniProtKB:Q8NHW5",
  "gene_name": "Putative ribosomal protein uL10-like"
}